{
  "gene": "UniProtKB:Q76EJ3",
  "gene_symbol": "SLC35D2",
  "gene_name": "UDP-N-acetylglucosamine_UDP-glucose_GDP-mannose transporter",
  "term_label": "Golgi apparatus",
  "term_id": "GO:0005794"
}